{
  "gene_symbol": "DCXR",
  "gene": "UniProtKB:Q7Z4W1",
  "term_label": "xylulose metabolic process",
  "gene_name": "L-xylulose reductase",
  "term_id": "GO:0005997"
}